{
  "gene_symbol": "OR8D1",
  "gene_name": "Olfactory receptor 8D1",
  "term_label": "olfactory receptor activity",
  "term_id": "GO:0004984",
  "gene": "UniProtKB:Q8WZ84"
}